{
  "term_id": "GO:0005829",
  "term_label": "cytosol",
  "gene": "UniProtKB:Q9NUV9",
  "gene_symbol": "GIMAP4",
  "gene_name": "GTPase IMAP family member 4"
}